{
  "gene_name": "Extracellular matrix protein 2",
  "gene_symbol": "ECM2",
  "term_label": "collagen V binding",
  "gene": "UniProtKB:O94769",
  "term_id": "GO:0070052"
}